{
  "term_label": "vesicle fusion with Golgi apparatus",
  "gene": "UniProtKB:O15155",
  "term_id": "GO:0048280",
  "gene_symbol": "BET1",
  "gene_name": "BET1 homolog"
}